{
  "gene_symbol": "Q6ZVU0",
  "term_id": "UNKNOWN:0001",
  "gene": "UniProtKB:Q6ZVU0",
  "term_label": "Unknown molecular function",
  "gene_name": "Putative uncharacterized protein FLJ42102"
}